galactose catabolic process via D-galactonate [GO:0033498] (biological process) Definition: The chemical reactions and pathways resulting in the breakdown of galactose, via the intermediate D-galactonate. Sources: GOC:mah, MetaCyc:GALDEG-PWY Also known as: galactose breakdown via D-galactonate, galactose catabolism via D-galactonate, galactose degradation via D-galactonate Relationships: is a type of GO:0019388